{
  "gene": "UniProtKB:Q96FE7",
  "gene_name": "Phosphoinositide-3-kinase-interacting protein 1",
  "gene_symbol": "PIK3IP1",
  "term_id": "GO:0051898",
  "term_label": "negative regulation of phosphatidylinositol 3-kinase/protein kinase B signal transduction"
}